uropod [GO:0001931] (cellular component) Definition: A membrane projection with related cytoskeletal components at the trailing edge of a cell in the process of migrating or being activated, found on the opposite side of the cell from the leading edge or immunological synapse, respectively. Relationships: is a type of GO:0120025; is part of cell trailing edge [GO:0031254] References: PMID:12714569, PMID:12787750 Sources: GOC:add, ISBN:0781735149 Also known as: uropodium, distal pole complex, retractile pole